{
  "gene_name": "Putative lung carcinoma-associated protein 10",
  "gene": "UniProtKB:Q71F78",
  "term_id": "UNKNOWN:0002",
  "gene_symbol": "LCA10",
  "term_label": "Unknown biological process"
}